{
  "gene": "UniProtKB:Q9BZI7",
  "term_id": "GO:0000184",
  "gene_symbol": "UPF3B",
  "term_label": "nuclear-transcribed mRNA catabolic process, nonsense-mediated decay",
  "gene_name": "Regulator of nonsense transcripts 3B"
}